regulation of cardioblast proliferation [GO:0003264] (biological process) Subtypes: GO:0003265, regulation of secondary heart field cardioblast proliferation [GO:0003266], GO:1905061, positive regulation of cardioblast proliferation [GO:1905062] Sources: GOC:mtg_heart Definition: Any process that modulates the frequency, rate or extent of cardioblast proliferation. A cardioblast is a cardiac precursor cell. It is a cell that has been committed to a cardiac fate, but will undergo more cell division rather than terminally differentiating. Relationships: is a type of regulation of cell proliferation involved in heart morphogenesis [GO:2000136]; regulates cardioblast proliferation [GO:0003263]